regulation of cell-cell adhesion mediated by integrin [GO:0033632] (biological process) Sources: GOC:add Subtypes: negative regulation of cell-cell adhesion mediated by integrin [GO:0033633], GO:0033634 Relationships: is a type of regulation of cell-cell adhesion [GO:0022407]; is a type of GO:0033628; regulates cell-cell adhesion mediated by integrin [GO:0033631] Also known as: regulation of cell-cell adhesion mediated by integrin complex Definition: Any process that modulates the frequency, rate, or extent of cell-cell adhesion mediated by integrin.